{
  "term_label": "Unknown biological process",
  "gene": "UniProtKB:A4D2P6",
  "gene_name": "Delphilin",
  "term_id": "UNKNOWN:0002",
  "gene_symbol": "GRID2IP"
}